{
  "gene_name": "Centrosomal protein of 19 kDa",
  "term_label": "microtubule anchoring at centrosome",
  "gene": "UniProtKB:Q96LK0",
  "term_id": "GO:0034454",
  "gene_symbol": "CEP19"
}